{
  "gene": "UniProtKB:Q04323",
  "gene_symbol": "UBXN1",
  "term_label": "negative regulation of protein ubiquitination",
  "gene_name": "UBX domain-containing protein 1",
  "term_id": "GO:0031397"
}